{
  "gene_name": "G antigen 12J",
  "gene_symbol": "GAGE12J",
  "term_id": "UNKNOWN:0003",
  "gene": "UniProtKB:A6NER3",
  "term_label": "Unknown cellular component"
}